{
  "term_label": "RNA polymerase II cis-regulatory region sequence-specific DNA binding",
  "gene_symbol": "ZIC3",
  "gene_name": "Zinc finger protein ZIC 3",
  "term_id": "GO:0000978",
  "gene": "UniProtKB:O60481"
}